desmosome disassembly [GO:0035921] (biological process) Definition: The controlled breakdown of a desmosome. A desmosome is a patch-like intercellular junction found in vertebrate tissues, consisting of parallel zones of two cell membranes, separated by an space of 25-35 nm, and having dense fibrillar plaques in the subjacent cytoplasm. References: PMID:9182671 Sources: GOC:BHF, GOC:vk, ISBN:0198506732 Relationships: is a type of desmosome organization [GO:0002934]; is a type of GO:0150147 Also known as: desmosome dissociation